hydrolase activity, acting on acid halide bonds, in C-halide compounds [GO:0019120] (molecular function) Sources: EC:3.8.1.- Subtypes: N-ethylammeline chlorohydrolase activity [GO:0016217], (S)-2-haloacid dehalogenase activity [GO:0018784], haloacetate dehalogenase activity [GO:0018785], haloalkane dehalogenase activity [GO:0018786], 4-chlorobenzoyl-CoA dehalogenase activity [GO:0018787], atrazine chlorohydrolase activity [GO:0018788], (R)-2-haloacid dehalogenase activity [GO:0033975], 2-haloacid dehalogenase (configuration-inverting) activity [GO:0033976], GO:0033977, 4-chlorobenzoate dehalogenase activity [GO:0047576], alkylhalidase activity [GO:0047651] Definition: Catalysis of the hydrolysis of any acid halide bond in substances containing halogen atoms in organic linkage. Relationships: is_a GO:0016824